arabinoxylan binding [GO:2001068] (molecular function) Sources: GOC:mengo_curators Relationships: is_a xylan binding [GO:2001062] Definition: Binding to arabinoxylan.